{
  "gene": "UniProtKB:Q9H2C5",
  "gene_symbol": "OR52A5",
  "gene_name": "Olfactory receptor 52A5",
  "term_label": "plasma membrane",
  "term_id": "GO:0005886"
}